{
  "gene_name": "Protein FAM83D",
  "gene_symbol": "FAM83D",
  "term_label": "protein localization to mitotic spindle",
  "term_id": "GO:1902480",
  "gene": "UniProtKB:Q9H4H8"
}